{
  "gene_symbol": "MBD1",
  "term_id": "GO:0008327",
  "term_label": "methyl-CpG binding",
  "gene_name": "Methyl-CpG-binding domain protein 1",
  "gene": "UniProtKB:Q9UIS9"
}